{
  "gene": "UniProtKB:Q53FT3",
  "term_id": "GO:0005634",
  "term_label": "nucleus",
  "gene_symbol": "HIKESHI",
  "gene_name": "Protein Hikeshi"
}